negative regulation of Rho protein signal transduction [GO:0035024] (biological process) Sources: GOC:bf Definition: Any process that stops, prevents, or reduces the frequency, rate or extent of Rho protein signal transduction. Also known as: down regulation of Rho protein signal transduction, down-regulation of Rho protein signal transduction, downregulation of Rho protein signal transduction, inhibition of Rho protein signal transduction Relationships: is a type of regulation of Rho protein signal transduction [GO:0035023]; is a type of GO:0051058; negatively regulates GO:0007266